glucosamine kinase activity [GO:0047931] (molecular function) Definition: Catalysis of the reaction: ATP + D-glucosamine = ADP + D-glucosamine 6-phosphate + H+. Sources: RHEA:10948 Also known as: ATP:2-amino-2-deoxy-D-glucose-6-phosphotransferase activity, ATP:D-glucosamine phosphotransferase activity, aminodeoxyglucose kinase activity, glucosamine kinase (phosphorylating) Relationships: is a type of GO:0016301; is a type of phosphotransferase activity, alcohol group as acceptor [GO:0016773]